{
  "gene": "UniProtKB:Q9NTN3",
  "gene_symbol": "SLC35D1",
  "term_label": "UDP-N-acetylgalactosamine transmembrane transporter activity",
  "term_id": "GO:0005463",
  "gene_name": "Nucleotide sugar transporter SLC35D1"
}